negative regulation of hair follicle maturation [GO:0048817] (biological process) Also known as: down regulation of hair follicle maturation, down-regulation of hair follicle maturation, downregulation of hair follicle maturation, inhibition of hair follicle maturation Subtypes: negative regulation of timing of catagen [GO:0051796], negative regulation of timing of anagen [GO:0051886], negative regulation of timing of exogen [GO:0051889] Sources: GOC:devbiol Definition: Any process that stops, prevents, or reduces the frequency, rate or extent of hair follicle maturation. Relationships: is_a regulation of hair follicle maturation [GO:0048819]; is a type of negative regulation of hair follicle development [GO:0051799]; negatively regulates hair follicle maturation [GO:0048820]